'de novo' L-methionine biosynthetic process [GO:0071266] (BP) Also known as: 'de novo' L-methionine anabolism, 'de novo' L-methionine biosynthesis, 'de novo' L-methionine formation, 'de novo' L-methionine synthesis Sources: GOC:ecd Relationships: is a type of L-methionine biosynthetic process [GO:0071265] Definition: The chemical reactions and pathways resulting in the formation of L-methionine, the L-enantiomer of (2S)-2-amino-4-(methylsulfanyl)butanoic acid, from simpler components. Subtypes: L-methionine biosynthetic process from L-homoserine via cystathionine [GO:0019279], L-methionine biosynthetic process from L-homoserine via O-phospho-L-homoserine and cystathionine [GO:0019283]